{
  "gene_symbol": "MRAP",
  "gene_name": "Melanocortin-2 receptor accessory protein",
  "gene": "UniProtKB:Q8TCY5",
  "term_label": "type 1 melanocortin receptor binding",
  "term_id": "GO:0070996"
}